endocrine process [GO:0050886] (biological process) Also known as: endocrine physiological process, endocrine physiology Definition: The process that involves the secretion of or response to endocrine hormones. An endocrine hormone is a hormone released into the circulatory system. Sources: ISBN:0721662544 Relationships: is a type of system process [GO:0003008] Regulation: regulated by GO:0044060 Subtypes: GO:0001990